{
  "term_label": "calcium-dependent activation of synaptic vesicle fusion",
  "gene": "UniProtKB:O00445",
  "gene_name": "Synaptotagmin-5",
  "gene_symbol": "SYT5",
  "term_id": "GO:0099502"
}